{
  "gene_symbol": "PRAMEF19",
  "term_id": "GO:0031462",
  "term_label": "Cul2-RING ubiquitin ligase complex",
  "gene": "UniProtKB:Q5SWL8",
  "gene_name": "PRAME family member 19"
}